{
  "gene_name": "Striated muscle preferentially expressed protein kinase",
  "gene": "UniProtKB:Q15772",
  "term_id": "GO:0004672",
  "term_label": "protein kinase activity",
  "gene_symbol": "SPEG"
}